{
  "gene_symbol": "ATP6AP2",
  "term_id": "GO:0009897",
  "gene": "UniProtKB:O75787",
  "gene_name": "Renin receptor",
  "term_label": "external side of plasma membrane"
}